{
  "term_id": "UNKNOWN:0003",
  "gene": "UniProtKB:Q01085",
  "gene_name": "Nucleolysin TIAR",
  "term_label": "Unknown cellular component",
  "gene_symbol": "TIAL1"
}